{
  "gene_symbol": "TPRX2",
  "term_id": "GO:0160021",
  "term_label": "maternal-to-zygotic transition of gene expression",
  "gene": "UniProtKB:P0DV77",
  "gene_name": "Tetrapeptide repeat homeobox protein 2"
}